{
  "gene_name": "Lymphocyte antigen 6E",
  "term_label": "plasma membrane",
  "term_id": "GO:0005886",
  "gene_symbol": "LY6E",
  "gene": "UniProtKB:Q16553"
}